{
  "gene_symbol": "RP9",
  "term_id": "UNKNOWN:0001",
  "gene_name": "Retinitis pigmentosa 9 protein",
  "term_label": "Unknown molecular function",
  "gene": "UniProtKB:Q8TA86"
}